{
  "term_id": "GO:0006888",
  "gene_name": "Protein TEX261",
  "term_label": "endoplasmic reticulum to Golgi vesicle-mediated transport",
  "gene": "UniProtKB:Q6UWH6",
  "gene_symbol": "TEX261"
}